{
  "gene_symbol": "OR5T1",
  "term_label": "Unknown cellular component",
  "term_id": "UNKNOWN:0003",
  "gene_name": "Olfactory receptor 5T1",
  "gene": "UniProtKB:Q8NG75"
}